3-hydroxyaspartate aldolase activity [GO:0047562] (molecular function) Also known as: erythro-3-hydroxy-L(s)-aspartate glyoxylate-lyase activity, erythro-3-hydroxy-Ls-aspartate glyoxylate-lyase (glycine-forming), erythro-3-hydroxy-Ls-aspartate glyoxylate-lyase activity, erythro-beta-hydroxyaspartate aldolase activity, erythro-beta-hydroxyaspartate glycine-lyase activity Definition: Catalysis of the reaction: (3R)-3-hydroxy-L-aspartate = glycine + glyoxylate. Relationships: is a type of oxo-acid-lyase activity [GO:0016833] Sources: EC:4.1.3.14, RHEA:14377